{
  "term_label": "Unknown molecular function",
  "term_id": "UNKNOWN:0001",
  "gene": "UniProtKB:Q92629",
  "gene_name": "Delta-sarcoglycan",
  "gene_symbol": "SGCD"
}